beta-glucoside kinase activity [GO:0047700] (molecular function) Relationships: is a type of GO:0016301; is a type of GO:0016773 Also known as: b-glucoside kinase activity, ATP:cellobiose 6-phosphotransferase activity, beta-D-glucoside kinase (phosphorylating) Sources: EC:2.7.1.85, MetaCyc:BETA-GLUCOSIDE-KINASE-RXN Definition: Catalysis of the reaction: ATP + cellobiose = ADP + 6-phospho-beta-D-glucosyl-(1,4)-D-glucose.